{
  "term_label": "7-methylguanosine mRNA capping",
  "gene_symbol": "CMTR2",
  "term_id": "GO:0006370",
  "gene_name": "Cap-specific mRNA (nucleoside-2'-O-)-methyltransferase 2",
  "gene": "UniProtKB:Q8IYT2"
}